{
  "gene_symbol": "CCL13",
  "gene_name": "C-C motif chemokine 13",
  "term_label": "chemokine-mediated signaling pathway",
  "gene": "UniProtKB:Q99616",
  "term_id": "GO:0070098"
}